{
  "gene_symbol": "RGR",
  "gene_name": "RPE-retinal G protein-coupled receptor",
  "term_id": "GO:0071482",
  "term_label": "cellular response to light stimulus",
  "gene": "UniProtKB:P47804"
}